{
  "term_label": "endomembrane system",
  "term_id": "GO:0012505",
  "gene_symbol": "RABL3",
  "gene": "UniProtKB:Q5HYI8",
  "gene_name": "Rab-like protein 3"
}